{
  "gene_symbol": "CD93",
  "gene_name": "Complement component C1q receptor",
  "gene": "UniProtKB:Q9NPY3",
  "term_label": "plasma membrane",
  "term_id": "GO:0005886"
}